{
  "gene_symbol": "CHAF1B",
  "term_label": "Unknown molecular function",
  "gene": "UniProtKB:Q13112",
  "gene_name": "Chromatin assembly factor 1 subunit B",
  "term_id": "UNKNOWN:0001"
}